{
  "term_id": "GO:0000132",
  "gene": "UniProtKB:Q14203",
  "gene_symbol": "DCTN1",
  "term_label": "establishment of mitotic spindle orientation",
  "gene_name": "Dynactin subunit 1"
}